response to iron ion starvation [GO:1990641] (biological process) References: PMID:16208485 Relationships: is a type of response to metal ion starvation [GO:0180055] Definition: Any process that results in a change in state or activity of a cell or an organism (in terms of movement, secretion, enzyme production, gene expression, etc.) as a result of a starvation stimulus, deprivation of iron ion.